{
  "term_label": "cytokine-mediated signaling pathway",
  "gene": "UniProtKB:Q9NSE2",
  "gene_symbol": "CISH",
  "term_id": "GO:0019221",
  "gene_name": "Cytokine-inducible SH2-containing protein"
}